hydroxylamine oxidoreductase activity [GO:0033740] (molecular function) Relationships: is a type of oxidoreductase activity, acting on other nitrogenous compounds as donors, cytochrome as acceptor [GO:0016662] Definition: Catalysis of the reaction: hydroxylamine + 3 Fe(III)-[cytochrome c] = nitric oxide + 3 Fe(II)-[cytochrome c] + 3 H+. Sources: RHEA:45036